{
  "gene_name": "Tubulin beta-3 chain",
  "term_label": "axon guidance",
  "gene_symbol": "TUBB3",
  "gene": "UniProtKB:Q13509",
  "term_id": "GO:0007411"
}